endoplasmic reticulum-endosome tether activity [GO:0170016] (molecular function) Relationships: is a type of endoplasmic reticulum-organelle membrane tether activity [GO:0170009] Definition: The binding activity of a molecule that brings together an endosome and an ER membrane either via membrane lipid binding or by interacting with an endosome protein, to establish and facilitate organelle exchange. References: PMID:33124732